{
  "term_label": "immunoglobulin complex",
  "gene_symbol": "IGLV10-54",
  "term_id": "GO:0019814",
  "gene_name": "Immunoglobulin lambda variable 10-54",
  "gene": "UniProtKB:A0A075B6I4"
}